{
  "gene": "UniProtKB:Q9HAW7",
  "gene_name": "UDP-glucuronosyltransferase 1A7",
  "term_label": "UDP-glycosyltransferase activity",
  "gene_symbol": "UGT1A7",
  "term_id": "GO:0008194"
}